{
  "gene": "UniProtKB:Q9H0A3",
  "gene_symbol": "TMEM191A",
  "term_label": "Unknown cellular component",
  "gene_name": "Transmembrane protein 191A",
  "term_id": "UNKNOWN:0003"
}